{
  "term_label": "cytosol",
  "gene_symbol": "GART",
  "term_id": "GO:0005829",
  "gene": "UniProtKB:P22102",
  "gene_name": "Trifunctional purine biosynthetic protein adenosine-3"
}